negative regulation of microglial cell mediated cytotoxicity [GO:1904150] (biological process) Relationships: is a type of GO:0001911; is a type of GO:0002887; is a type of regulation of microglial cell mediated cytotoxicity [GO:1904149]; negatively regulates microglial cell mediated cytotoxicity [GO:0090634] Definition: Any process that stops, prevents or reduces the frequency, rate or extent of microglial cell mediated cytotoxicity. Also known as: down regulation of microglial cell mediated cytotoxicity, down-regulation of microglial cell mediated cytotoxicity, downregulation of microglial cell mediated cytotoxicity, inhibition of microglial cell mediated cytotoxicity References: PMID:19100238 Sources: GOC:BHF, GOC:TermGenie, GOC:nc, GO_REF:0000058